{
  "term_label": "regulation of intracellular signal transduction",
  "term_id": "GO:1902531",
  "gene_symbol": "SASH3",
  "gene_name": "SAM and SH3 domain-containing protein 3",
  "gene": "UniProtKB:O75995"
}